{
  "gene_symbol": "BAG5",
  "term_id": "GO:0005634",
  "gene": "UniProtKB:Q9UL15",
  "gene_name": "BAG family molecular chaperone regulator 5",
  "term_label": "nucleus"
}